{
  "gene": "UniProtKB:Q96N11",
  "term_label": "Unknown biological process",
  "gene_name": "Integrator complex subunit 15",
  "term_id": "UNKNOWN:0002",
  "gene_symbol": "INTS15"
}